{
  "term_label": "Unknown biological process",
  "gene": "UniProtKB:Q96GQ5",
  "term_id": "UNKNOWN:0002",
  "gene_symbol": "RUSF1",
  "gene_name": "RUS family member 1"
}